{
  "term_id": "UNKNOWN:0001",
  "gene": "UniProtKB:Q92844",
  "gene_symbol": "TANK",
  "term_label": "Unknown molecular function",
  "gene_name": "TRAF family member-associated NF-kappa-B activator"
}